{
  "gene": "UniProtKB:A0JLT2",
  "gene_name": "Mediator of RNA polymerase II transcription subunit 19",
  "term_label": "Unknown molecular function",
  "term_id": "UNKNOWN:0001",
  "gene_symbol": "MED19"
}